{
  "gene_name": "Probable G-protein coupled receptor 152",
  "term_id": "GO:0004930",
  "gene_symbol": "GPR152",
  "term_label": "G protein-coupled receptor activity",
  "gene": "UniProtKB:Q8TDT2"
}